{
  "term_id": "GO:0031681",
  "gene": "UniProtKB:P63218",
  "gene_name": "Guanine nucleotide-binding protein G(I)_G(S)_G(O) subunit gamma-5",
  "term_label": "G-protein beta-subunit binding",
  "gene_symbol": "GNG5"
}